{
  "gene": "UniProtKB:Q6T4R5",
  "gene_symbol": "NHS",
  "term_label": "Unknown cellular component",
  "term_id": "UNKNOWN:0003",
  "gene_name": "Actin remodeling regulator NHS"
}